imaginal disc-derived wing morphogenesis [GO:0007476] (biological process) Also known as: wing morphogenesis Relationships: is a type of imaginal disc-derived appendage morphogenesis [GO:0035114]; is a type of post-embryonic appendage morphogenesis [GO:0035120]; is part of GO:0007472 Sources: GOC:bf, GOC:mtg_sensu Definition: The process in which the anatomical structures of the imaginal disc-derived wing are generated and organized. The wing is an appendage modified for flying.